{
  "gene_name": "General transcription factor II-I repeat domain-containing protein 2B",
  "term_label": "Unknown biological process",
  "gene": "UniProtKB:Q6EKJ0",
  "gene_symbol": "GTF2IRD2B",
  "term_id": "UNKNOWN:0002"
}